L-pipecolate dehydrogenase activity [GO:0050030] (molecular function) Sources: EC:1.5.99.3, MetaCyc:L-PIPECOLATE-DEHYDROGENASE-RXN Definition: Catalysis of the reaction: L-pipecolate + acceptor = delta1-piperideine-6-carboxylate + reduced acceptor. Delta1-piperideine-6-carboxylate is also known as 2,3,4,5-tetrahydropyridine-2-carboxylate. Relationships: is a type of oxidoreductase activity, acting on the CH-NH group of donors [GO:0016645] Also known as: L-pipecolate:(acceptor) 1,6-oxidoreductase activity, L-pipecolate:acceptor 1,6-oxidoreductase activity